{
  "gene": "UniProtKB:Q8NDZ6",
  "term_label": "Unknown molecular function",
  "gene_symbol": "TMEM161B",
  "term_id": "UNKNOWN:0001",
  "gene_name": "Transmembrane protein 161B"
}